syntrophin complex [GO:0016013] (cellular component) Definition: A protein complex that includes alpha-, beta1-, beta2-syntrophins and syntrophin-like proteins; the syntrophin complex binds to the second half of the carboxy-terminal domain of dystrophin; also associates with neuronal nitric oxide synthase. References: PMID:23263165 Relationships: is a type of plasma membrane protein complex [GO:0098797]; is part of dystrophin-associated glycoprotein complex [GO:0016010] Also known as: nitric oxide synthase-dystrophin complex, skeletal muscle